{
  "term_label": "RNA polymerase II cis-regulatory region sequence-specific DNA binding",
  "term_id": "GO:0000978",
  "gene": "UniProtKB:Q7L2R6",
  "gene_symbol": "ZNF765",
  "gene_name": "Zinc finger protein 765"
}